{
  "term_id": "GO:0005634",
  "gene": "UniProtKB:Q7Z2Z1",
  "gene_name": "Treslin",
  "term_label": "nucleus",
  "gene_symbol": "TICRR"
}